{
  "gene_name": "Estrogen receptor beta",
  "gene": "UniProtKB:Q92731",
  "term_id": "GO:0004879",
  "term_label": "nuclear receptor activity",
  "gene_symbol": "ESR2"
}